codeinone reductase (NADPH) activity [GO:0047036] (molecular function) Relationships: is_a oxidoreductase activity, acting on the CH-OH group of donors, NAD or NADP as acceptor [GO:0016616] Definition: Catalysis of the reaction: codeine + NADP+ = codeinone + H+ + NADPH. Sources: EC:1.1.1.247, RHEA:19209 Also known as: codeine:NADP+ oxidoreductase activity